{
  "term_label": "RNA binding",
  "gene_symbol": "RPS27L",
  "gene_name": "Ribosomal protein eS27-like",
  "term_id": "GO:0003723",
  "gene": "UniProtKB:Q71UM5"
}